{
  "gene_symbol": "ZNF355P",
  "gene_name": "Putative zinc finger protein 355P",
  "gene": "UniProtKB:Q9NSJ1",
  "term_id": "GO:0000981",
  "term_label": "DNA-binding transcription factor activity, RNA polymerase II-specific"
}